{
  "gene_symbol": "ZNF213",
  "gene_name": "Zinc finger protein 213",
  "term_label": "DNA-binding transcription factor activity, RNA polymerase II-specific",
  "gene": "UniProtKB:O14771",
  "term_id": "GO:0000981"
}